{
  "gene_name": "E3 ubiquitin-protein ligase PDZRN3",
  "gene_symbol": "PDZRN3",
  "gene": "UniProtKB:Q9UPQ7",
  "term_id": "GO:0016567",
  "term_label": "protein ubiquitination"
}